detection of electrical stimulus involved in sensory perception of pain [GO:0050967] (biological process) Definition: The series of events that contribute to the perception of pain in which an electrical stimulus is received and converted into a molecular signal. Sources: GOC:ai, GOC:dos, GOC:dph, GOC:tb Also known as: perception of pain, detection of electrical stimulus, perception of pain, sensory detection of electrical stimulus, perception of pain, sensory transduction of electrical stimulus, detection of electrical stimulus during sensory perception of pain, sensory detection of electrical stimulus during perception of pain, sensory transduction of electrical stimulus during perception of pain Relationships: is a type of detection of electrical stimulus involved in sensory perception [GO:0050963]; is a type of GO:0062149